{
  "gene": "UniProtKB:Q99985",
  "term_label": "axon guidance",
  "gene_symbol": "SEMA3C",
  "term_id": "GO:0007411",
  "gene_name": "Semaphorin-3C"
}